{
  "gene_symbol": "WFDC3",
  "term_label": "serine-type endopeptidase inhibitor activity",
  "gene_name": "WAP four-disulfide core domain protein 3",
  "gene": "UniProtKB:Q8IUB2",
  "term_id": "GO:0004867"
}